{
  "gene_symbol": "ATG16L1",
  "gene_name": "Autophagy-related protein 16-1",
  "term_id": "GO:0000045",
  "term_label": "autophagosome assembly",
  "gene": "UniProtKB:Q676U5"
}